secretory granule-lysosome fusion [GO:0160156] (biological process) References: PMID:29066608, PMID:35452619 Relationships: is a type of GO:0006906; is part of crinophagy [GO:0160155] Definition: The cellular process that results in the fusion of secretory granules with lysosomes to form crinosomes.